{
  "term_id": "GO:0030317",
  "gene_symbol": "EFCAB9",
  "gene_name": "EF-hand calcium-binding domain-containing protein 9",
  "gene": "UniProtKB:A8MZ26",
  "term_label": "flagellated sperm motility"
}